{
  "gene_name": "MOB kinase activator 3A",
  "gene": "UniProtKB:Q96BX8",
  "term_label": "cytoplasm",
  "gene_symbol": "MOB3A",
  "term_id": "GO:0005737"
}